dipeptide transport [GO:0042938] (biological process) Regulation: regulated by regulation of dipeptide transport [GO:0090089]; negatively regulated by negative regulation of dipeptide transport [GO:2000879]; RO_0002213 by positive regulation of dipeptide transport [GO:2000880] Definition: The directed movement of a dipeptide, a combination of two amino acids by means of a peptide (-CO-NH-) link, into, out of or within a cell, or between cells, by means of some agent such as a transporter or pore. Subtypes: p-aminobenzoyl-glutamate transport [GO:0015814], dipeptide transmembrane transport [GO:0035442], chrysobactin transport [GO:0042932] Sources: GOC:jl Relationships: is a type of oligopeptide transport [GO:0006857]